polar tube anchoring disc [GO:0160202] (cellular component) References: PMID:16005007, PMID:19673893 Relationships: is_a cellular anatomical structure [GO:0110165] Definition: A structural component of the microsporidian spore's invasion apparatus that is located at the anterior end of the spore and serves to attach the polar tube to the inside of the spore wall.